sleep homeostasis [GO:0160060] (BP) References: PMID:30509635 Definition: A homeostatic process in which the drive for sleep increases sleep propensity with prolonged wakefulness. Relationships: is a type of multicellular organismal-level homeostasis [GO:0048871]